{
  "gene_symbol": "TSPAN16",
  "term_id": "UNKNOWN:0002",
  "gene_name": "Tetraspanin-16",
  "term_label": "Unknown biological process",
  "gene": "UniProtKB:Q9UKR8"
}